phosphatidylinositol-3,4-bisphosphate phosphatase activity [GO:0106017] (molecular function) Relationships: is_a GO:0034593 Subtypes: phosphatidylinositol-3,4-bisphosphate 4-phosphatase activity [GO:0016316], GO:0051800 Sources: GOC:hjd Definition: Catalysis of the reaction: 1-phosphatidyl-1D-myo-inositol 3,4-bisphosphate + H2O = 1-phosphatidyl-1D-myo-inositol phosphate + phosphate.